{
  "gene_symbol": "ANKRD20A4P",
  "gene": "UniProtKB:Q4UJ75",
  "term_label": "Unknown cellular component",
  "gene_name": "Putative ankyrin repeat domain-containing protein 20A4",
  "term_id": "UNKNOWN:0003"
}